cellular response to alkaline pH [GO:0071469] (biological process) Also known as: cellular response to alkalinity, cellular response to basic pH Definition: Any process that results in a change in state or activity of a cell (in terms of movement, secretion, enzyme production, gene expression, etc.) as a result of a pH stimulus with pH > 7. pH is a measure of the acidity or basicity of an aqueous solution. Regulation: regulated by regulation of cellular response to alkaline pH [GO:1900067]; negatively regulated by negative regulation of cellular response to alkaline pH [GO:1900068] Relationships: is a type of GO:0010446; is a type of cellular response to pH [GO:0071467] Sources: GOC:go_curators, GOC:mah, Wikipedia:PH